{
  "gene_name": "Kinesin-like protein KIF13B",
  "term_id": "GO:0005737",
  "gene": "UniProtKB:Q9NQT8",
  "gene_symbol": "KIF13B",
  "term_label": "cytoplasm"
}